vitamin A metabolic process [GO:0006776] (biological process) Regulation: regulated by regulation of vitamin A metabolic process [GO:1901738] Subtypes: vitamin A biosynthetic process [GO:0035238] References: PMID:1503811 Sources: GOC:jl Also known as: vitamin A metabolism Definition: The chemical reactions and pathways involving any of the vitamin A compounds, retinol, retinal (retinaldehyde) and retinoic acid, all of which are derivatives of beta-carotene. Relationships: is a type of retinoid metabolic process [GO:0001523]